{
  "term_label": "lysosomal membrane",
  "gene": "UniProtKB:O60931",
  "gene_symbol": "CTNS",
  "gene_name": "Cystinosin",
  "term_id": "GO:0005765"
}